spinal sensory neuron axon guidance [GO:0097375] (biological process) Sources: CL:0009000, GOC:pr, GOC:yaf Definition: The process in which the migration of an axon growth cone of a spinal sensory neuron is directed to a specific target site in response to a combination of attractive and repulsive cues. A spinal sensory neuron is a sensory neuron that project to the spinal cord. Relationships: is a type of sensory neuron axon guidance [GO:0097374]